{
  "gene_name": "Retinoic acid receptor responder protein 2",
  "term_id": "GO:0050994",
  "gene_symbol": "RARRES2",
  "term_label": "regulation of lipid catabolic process",
  "gene": "UniProtKB:Q99969"
}